sulfatide binding [GO:0120146] (molecular function) References: PMID:21525289, PMID:22619219, PMID:22977233, PMID:23574804, PMID:29497057, PMID:3549017 Sources: GOC:krc, Wikipedia:Sulfatide Definition: Binding to sulfatide, also known as 3-O-sulfogalactosylceramide, SM4, or sulfated galactocerebroside. Sulfatide is a class of sulfoglycolipid, which are glycolipids that contain a sulfate group. Relationships: is a type of glycolipid binding [GO:0051861] Also known as: 3-O-sulfogalactosylceramide binding, SM4 binding, sulfated galactocerebroside binding